beta-alanine biosynthetic process [GO:0019483] (biological process) Sources: GOC:jl, ISBN:0198506732 Definition: The chemical reactions and pathways resulting in the formation of beta-alanine (3-aminopropanoic acid), an achiral amino acid and an isomer of alanine. It occurs free (e.g. in brain) and in combination (e.g. in pantothenate) but it is not a constituent of proteins. Relationships: is a type of amino acid biosynthetic process [GO:0008652]; is a type of GO:0019482; is a type of non-proteinogenic amino acid biosynthetic process [GO:0170043] Subtypes: beta-alanine biosynthetic process via 1,3 diaminopropane [GO:0033394], beta-alanine biosynthetic process via 3-hydroxypropionate [GO:0033395], beta-alanine biosynthetic process via 3-ureidopropionate [GO:0033396] Also known as: beta-alanine anabolism, beta-alanine biosynthesis, beta-alanine formation, beta-alanine synthesis